{
  "gene_name": "Protein furry homolog-like",
  "gene": "UniProtKB:O94915",
  "term_label": "cell morphogenesis",
  "term_id": "GO:0000902",
  "gene_symbol": "FRYL"
}